{
  "term_id": "GO:0004867",
  "term_label": "serine-type endopeptidase inhibitor activity",
  "gene_name": "Histidine-rich glycoprotein",
  "gene": "UniProtKB:P04196",
  "gene_symbol": "HRG"
}